{
  "term_id": "GO:1900029",
  "gene": "UniProtKB:Q8TE67",
  "gene_name": "Epidermal growth factor receptor kinase substrate 8-like protein 3",
  "term_label": "positive regulation of ruffle assembly",
  "gene_symbol": "EPS8L3"
}